arabitol catabolic process [GO:0051157] (biological process) Subtypes: L-arabitol catabolic process [GO:0051158], D-arabitol catabolic process [GO:0051159] Definition: The chemical reactions and pathways resulting in the breakdown of arabitol, the pentitol derived from arabinose or lyxose by reduction of the aldehyde group. Sources: ISBN:0198506732 Also known as: arabitol breakdown, arabitol catabolism, arabitol degradation, arabitol utilization Relationships: is_a pentitol catabolic process [GO:0019527]